negative regulation of toll-like receptor 21 signaling pathway [GO:2000444] (biological process) Sources: GOC:obol Also known as: negative regulation of TLR21 signaling pathway, negative regulation of toll-like receptor 21 signalling pathway Definition: Any process that stops, prevents or reduces the frequency, rate or extent of toll-like receptor 21 signaling pathway. Relationships: is a type of negative regulation of toll-like receptor signaling pathway [GO:0034122]; is a type of regulation of toll-like receptor 21 signaling pathway [GO:2000443]; RO_0002212 GO:0035682